{
  "gene": "UniProtKB:Q6ZRP7",
  "term_label": "flavin-dependent sulfhydryl oxidase activity",
  "gene_name": "Sulfhydryl oxidase 2",
  "gene_symbol": "QSOX2",
  "term_id": "GO:0016971"
}